{
  "term_label": "Unknown biological process",
  "term_id": "UNKNOWN:0002",
  "gene_symbol": "C4orf17",
  "gene_name": "Uncharacterized protein C4orf17",
  "gene": "UniProtKB:Q53FE4"
}